L-alanine metabolic process [GO:0042851] (biological process) Also known as: L-alanine metabolism Definition: The chemical reactions and pathways involving L-alanine, the L-enantiomer of 2-aminopropanoic acid, i.e. (2S)-2-aminopropanoic acid. Sources: GOC:jl, GOC:jsg, GOC:mah Subtypes: beta-alanine catabolic process to L-alanine [GO:0019485], L-alanine biosynthetic process [GO:0042852], L-alanine catabolic process [GO:0042853] Relationships: is a type of alanine metabolic process [GO:0006522]; is_a L-amino acid metabolic process [GO:0170033]; is a type of proteinogenic amino acid metabolic process [GO:0170039]